entry of intact viral capsid into host nucleus through nuclear pore complex [GO:0075505] (biological process) Note: This mechanism is used by viruses with capsids small enough to cross the nuclear pore complex, such as the single-stranded (ss) DNA viruses Parvoviridae, Circoviridae and Geminiviridae. References: PMID:22929056 Sources: VZ:989 Definition: Viral penetration into the host nucleus where a viral capsid passes intact through the host nuclear pore complex (NPC). Relationships: is a type of viral penetration into host nucleus [GO:0075732]